U12 snRNP [GO:0005693] (cellular component) Definition: A ribonucleoprotein complex that contains small nuclear RNA U12, a heptameric ring of Sm proteins, as well as several proteins that are unique to the U12 snRNP, most of which remain associated with the U12 snRNA both while the U12 snRNP is free or assembled into a series of spliceosomal complexes. Relationships: is_a GO:0097525 Sources: GOC:krc, GOC:mah, ISBN:0879695897 Also known as: snRNP U12